branched-chain amino acid transport [GO:0015803] (biological process) Sources: GOC:ai, GOC:bf Definition: The directed movement of branched-chain amino acids into, out of or within a cell, or between cells, by means of some agent such as a transporter or pore. Branched-chain amino acids are amino acids with a branched carbon skeleton without rings. Also known as: branched-chain aliphatic amino acid transport, branched-chain amino-acid anion transport, branched-chain amino-acid anions transport Relationships: is a type of GO:0046942; is a type of nitrogen compound transport [GO:0071705] Subtypes: isoleucine transport [GO:0015818], GO:0015820, valine transport [GO:0015829]